{
  "term_id": "GO:0006338",
  "gene": "UniProtKB:O95619",
  "term_label": "chromatin remodeling",
  "gene_symbol": "YEATS4",
  "gene_name": "YEATS domain-containing protein 4"
}